{
  "gene_name": "WD repeat domain phosphoinositide-interacting protein 2",
  "term_id": "GO:0030674",
  "gene": "UniProtKB:Q9Y4P8",
  "gene_symbol": "WIPI2",
  "term_label": "protein-macromolecule adaptor activity"
}